{
  "gene_symbol": "DSG3",
  "gene": "UniProtKB:P32926",
  "term_label": "cell-cell adhesion",
  "term_id": "GO:0098609",
  "gene_name": "Desmoglein-3"
}